{
  "term_id": "GO:0032426",
  "term_label": "stereocilium tip",
  "gene_name": "Harmonin",
  "gene": "UniProtKB:Q9Y6N9",
  "gene_symbol": "USH1C"
}